{
  "gene_symbol": "HOXC5",
  "term_label": "anterior/posterior pattern specification",
  "gene": "UniProtKB:Q00444",
  "gene_name": "Homeobox protein Hox-C5",
  "term_id": "GO:0009952"
}